(-)-secologanin biosynthetic process [GO:1900994] (biological process) Relationships: is a type of monoterpenoid biosynthetic process [GO:0016099]; is a type of aldehyde biosynthetic process [GO:0046184]; is a type of olefinic compound biosynthetic process [GO:0120255]; is a type of beta-glucoside biosynthetic process [GO:1901806] Definition: The chemical reactions and pathways resulting in the formation of (-)-secologanin. References: PMID:24104568 Sources: GOC:TermGenie, GOC:yaf Also known as: (-)-secologanin anabolism, (-)-secologanin biosynthesis, (-)-secologanin formation, (-)-secologanin synthesis